negative regulation of myeloid dendritic cell chemotaxis [GO:2000528] (biological process) Relationships: is a type of negative regulation of dendritic cell chemotaxis [GO:2000509]; is a type of regulation of myeloid dendritic cell chemotaxis [GO:2000527]; negatively regulates myeloid dendritic cell chemotaxis [GO:0002408] Sources: GOC:obol Definition: Any process that stops, prevents or reduces the frequency, rate or extent of myeloid dendritic cell chemotaxis.